{
  "gene_symbol": "MLH3",
  "term_id": "GO:0006298",
  "gene_name": "DNA mismatch repair protein Mlh3",
  "gene": "UniProtKB:Q9UHC1",
  "term_label": "mismatch repair"
}